{
  "gene": "UniProtKB:Q8N307",
  "gene_symbol": "MUC20",
  "term_id": "GO:0048012",
  "term_label": "hepatocyte growth factor receptor signaling pathway",
  "gene_name": "Mucin-20"
}